{
  "term_id": "GO:0005737",
  "gene": "UniProtKB:P84550",
  "gene_name": "SKI family transcriptional corepressor 1",
  "gene_symbol": "SKOR1",
  "term_label": "cytoplasm"
}